{
  "gene_symbol": "TSPAN17",
  "term_label": "Unknown biological process",
  "gene_name": "Tetraspanin-17",
  "gene": "UniProtKB:Q96FV3",
  "term_id": "UNKNOWN:0002"
}